FANCM-MHF complex [GO:0071821] (cellular component) Relationships: is a type of GO:0140513 References: PMID:20347428 Sources: GOC:mah, GOC:vw Definition: A protein complex contains the proteins FANCM and MHF, or their orthologs, plays an essential role in DNA remodeling, protects replication forks, and is conserved in eukaryotes.